{
  "term_id": "GO:1990075",
  "gene_symbol": "RP2",
  "gene_name": "Protein XRP2",
  "term_label": "periciliary membrane compartment",
  "gene": "UniProtKB:O75695"
}